{
  "term_label": "Unknown molecular function",
  "gene_name": "Uncharacterized protein C15orf32",
  "gene_symbol": "C15orf32",
  "term_id": "UNKNOWN:0001",
  "gene": "UniProtKB:Q32M92"
}